viral tegument [GO:0019033] (cellular component) Definition: A structure lying between the capsid and envelope of a virus, varying in thickness and often distributed asymmetrically. Relationships: is a type of virion component [GO:0044423] Sources: ISBN:0721662544